response to diamide [GO:0072737] (biological process) Relationships: is a type of GO:1901698 Also known as: response to N,N,N',N'-tetramethyldiazene-1,2-dicarboxamide Sources: GOC:mah Subtypes: cellular response to diamide [GO:0072738] Definition: Any process that results in a change in state or activity of a cell or an organism (in terms of movement, secretion, enzyme production, gene expression, etc.) as a result of a diamide (N,N,N',N'-tetramethyldiazene-1,2-dicarboxamide) stimulus.